{
  "gene_symbol": "UACA",
  "gene_name": "Uveal autoantigen with coiled-coil domains and ankyrin repeats",
  "term_id": "GO:0005634",
  "gene": "UniProtKB:Q9BZF9",
  "term_label": "nucleus"
}